{
  "term_id": "GO:0005737",
  "gene_name": "Tyrosine-protein phosphatase non-receptor type 3",
  "term_label": "cytoplasm",
  "gene": "UniProtKB:P26045",
  "gene_symbol": "PTPN3"
}